{
  "gene_name": "Dual adapter for phosphotyrosine and 3-phosphotyrosine and 3-phosphoinositide",
  "term_id": "GO:0005886",
  "term_label": "plasma membrane",
  "gene": "UniProtKB:Q9UN19",
  "gene_symbol": "DAPP1"
}